{
  "gene_name": "Valacyclovir hydrolase",
  "term_label": "Unknown biological process",
  "gene": "UniProtKB:Q86WA6",
  "term_id": "UNKNOWN:0002",
  "gene_symbol": "BPHL"
}